{
  "gene_name": "Toll-like receptor 9",
  "term_label": "toll-like receptor signaling pathway",
  "gene_symbol": "TLR9",
  "term_id": "GO:0002224",
  "gene": "UniProtKB:Q9NR96"
}